protein guanylyltransferase activity [GO:0044600] (molecular function) References: PMID:20651120 Sources: GOC:sp Definition: Catalysis of the reaction: GTP + protein = diphosphate + guanylyl-protein; mediates the addition of an guanylyl (guanosine 5'-monophosphate; GMP group) to specific residues of target proteins. Relationships: is a type of guanylyltransferase activity [GO:0070568]; is part of GO:0018260